{
  "term_id": "GO:0008284",
  "gene_name": "Fibroblast growth factor 16",
  "term_label": "positive regulation of cell population proliferation",
  "gene": "UniProtKB:O43320",
  "gene_symbol": "FGF16"
}